{
  "gene_name": "Tropomodulin-2",
  "term_label": "striated muscle thin filament",
  "gene_symbol": "TMOD2",
  "gene": "UniProtKB:Q9NZR1",
  "term_id": "GO:0005865"
}